{
  "gene": "UniProtKB:Q9UNH5",
  "gene_name": "Dual specificity protein phosphatase CDC14A",
  "term_label": "regulation of exit from mitosis",
  "gene_symbol": "CDC14A",
  "term_id": "GO:0007096"
}